antigen processing and presentation following phagocytosis [GO:0002747] (biological process) Sources: GOC:add, ISBN:0781735149 Relationships: is a type of antigen processing and presentation [GO:0019882] Definition: Antigen processing and presentation which is initiated by uptake of antigen via phagocytosis.